{
  "term_id": "UNKNOWN:0003",
  "gene_symbol": "USP17L23",
  "term_label": "Unknown cellular component",
  "gene": "UniProtKB:D6RBM5",
  "gene_name": "Putative ubiquitin carboxyl-terminal hydrolase 17-like protein 23"
}